{
  "gene": "UniProtKB:O43663",
  "gene_symbol": "PRC1",
  "term_label": "mitotic spindle midzone",
  "term_id": "GO:1990023",
  "gene_name": "Protein regulator of cytokinesis 1"
}